{
  "gene_symbol": "TMEM139",
  "term_label": "Unknown molecular function",
  "term_id": "UNKNOWN:0001",
  "gene_name": "Transmembrane protein 139",
  "gene": "UniProtKB:Q8IV31"
}